{
  "term_id": "GO:0003729",
  "gene_symbol": "DDX3Y",
  "gene_name": "ATP-dependent RNA helicase DDX3Y",
  "term_label": "mRNA binding",
  "gene": "UniProtKB:O15523"
}